{
  "gene_name": "Proline-rich protein 35",
  "gene_symbol": "PRR35",
  "gene": "UniProtKB:P0CG20",
  "term_id": "UNKNOWN:0001",
  "term_label": "Unknown molecular function"
}